{
  "term_label": "Unknown cellular component",
  "gene": "UniProtKB:Q9BQ66",
  "gene_name": "Keratin-associated protein 4-12",
  "gene_symbol": "KRTAP4-12",
  "term_id": "UNKNOWN:0003"
}